positive regulation of protein geranylgeranylation [GO:2000541] (biological process) Relationships: is a type of positive regulation of protein modification process [GO:0031401]; is a type of regulation of protein geranylgeranylation [GO:2000539]; positively regulates GO:0018344 Also known as: positive regulation of protein amino acid geranylgeranylation, positive regulation of C-terminal protein geranylgeranylation Definition: Any process that activates or increases the frequency, rate or extent of protein geranylgeranylation. Sources: GOC:obol